regulation of amyloid-beta formation [GO:1902003] (biological process) References: PMID:17098871 Sources: GOC:TermGenie, GOC:dph Also known as: regulation of beta-amyloid formation Definition: Any process that modulates the frequency, rate or extent of amyloid-beta formation. Subtypes: GO:1902004, negative regulation of amyloid-beta formation [GO:1902430] Relationships: is a type of regulation of amide metabolic process [GO:0034248]; is a type of regulation of amyloid precursor protein catabolic process [GO:1902991]; regulates amyloid-beta formation [GO:0034205]